{
  "term_label": "Unknown biological process",
  "gene_name": "Testis-specific gene 10 protein",
  "gene": "UniProtKB:Q9BZW7",
  "term_id": "UNKNOWN:0002",
  "gene_symbol": "TSGA10"
}